{
  "gene_name": "PAK4-inhibitor INKA1",
  "gene": "UniProtKB:Q96EL1",
  "gene_symbol": "INKA1",
  "term_id": "UNKNOWN:0002",
  "term_label": "Unknown biological process"
}